testosterone 16-beta-hydroxylase activity [GO:0062184] (molecular function) Relationships: is a type of steroid hydroxylase activity [GO:0008395] Definition: Catalysis of the reaction: O2 + reduced [NADPH--hemoprotein reductase] + testosterone = 16beta,17beta-dihydroxyandrost-4-en-3-one + H+ + H2O + oxidized [NADPH--hemoprotein reductase]. References: PMID:21289075 Sources: RHEA:46304